L-ascorbic acid biosynthetic process via UDP-alpha-D-glucuronate [GO:0090532] (biological process) Note: This pathway occurs in most vertebrates, although not in guinea pigs and primates, including humans. Relationships: is a type of L-ascorbic acid biosynthetic process [GO:0019853] References: PMID:11153268 Sources: GOC:yaf Definition: The chemical reactions and pathways resulting in the formation of L-ascorbic acid via the intermediate UDP-alpha-D-glucuronate. Also known as: L-ascorbic acid biosynthesis via UDP-alpha-D-glucuronate